{
  "term_id": "UNKNOWN:0001",
  "gene_symbol": "EPM2A",
  "gene": "UniProtKB:B3EWF7",
  "gene_name": "Laforin, isoform 9",
  "term_label": "Unknown molecular function"
}